{
  "term_id": "GO:0110104",
  "term_label": "mRNA alternative polyadenylation",
  "gene_name": "Cleavage and polyadenylation specificity factor subunit 6",
  "gene": "UniProtKB:Q16630",
  "gene_symbol": "CPSF6"
}